{
  "term_id": "GO:0006096",
  "gene_symbol": "GPI",
  "term_label": "glycolytic process",
  "gene_name": "Glucose-6-phosphate isomerase",
  "gene": "UniProtKB:P06744"
}